{
  "term_id": "UNKNOWN:0001",
  "gene": "UniProtKB:A6NJU9",
  "gene_name": "Nuclear pore complex-interacting protein family member B13",
  "term_label": "Unknown molecular function",
  "gene_symbol": "NPIPB13"
}